{
  "term_id": "GO:0005737",
  "gene_symbol": "PAK1",
  "gene": "UniProtKB:Q13153",
  "term_label": "cytoplasm",
  "gene_name": "Serine_threonine-protein kinase PAK 1"
}